{
  "gene_name": "Proto-oncogene c-Rel",
  "term_id": "GO:0045087",
  "term_label": "innate immune response",
  "gene_symbol": "REL",
  "gene": "UniProtKB:Q04864"
}